{
  "term_label": "plasma membrane",
  "term_id": "GO:0005886",
  "gene": "UniProtKB:Q99569",
  "gene_name": "Plakophilin-4",
  "gene_symbol": "PKP4"
}